{
  "term_label": "Unknown biological process",
  "gene_symbol": "THBS3",
  "gene_name": "Thrombospondin-3",
  "term_id": "UNKNOWN:0002",
  "gene": "UniProtKB:P49746"
}